negative regulation of intrinsic apoptotic signaling pathway in response to hydrogen peroxide [GO:1903751] (biological process) Definition: Any process that stops, prevents or reduces the frequency, rate or extent of intrinsic apoptotic signaling pathway in response to hydrogen peroxide. Subtypes: negative regulation of hydrogen peroxide-induced neuron intrinsic apoptotic signaling pathway [GO:1903384] Relationships: is a type of negative regulation of hydrogen peroxide-mediated programmed cell death [GO:1901299]; is a type of negative regulation of oxidative stress-induced intrinsic apoptotic signaling pathway [GO:1902176]; is a type of regulation of intrinsic apoptotic signaling pathway in response to hydrogen peroxide [GO:1903750]; negatively regulates GO:0036481 References: PMID:18681888 Sources: GOC:TermGenie, GO_REF:0000058 Also known as: down regulation of hydrogen peroxide-induced intrinsic apoptotic signaling pathway, down regulation of intrinsic apoptotic signaling pathway in response to H2O2, down regulation of intrinsic apoptotic signaling pathway in response to hydrogen peroxide, down-regulation of hydrogen peroxide-induced intrinsic apoptotic signaling pathway, down-regulation of intrinsic apoptotic signaling pathway in response to H2O2, down-regulation of intrinsic apoptotic signaling pathway in response to hydrogen peroxide, downregulation of hydrogen peroxide-induced intrinsic apoptotic signaling pathway, downregulation of intrinsic apoptotic signaling pathway in response to H2O2, downregulation of intrinsic apoptotic signaling pathway in response to hydrogen peroxide, negative regulation of hydrogen peroxide-induced intrinsic apoptotic signaling pathway, negative regulation of intrinsic apoptotic signaling pathway in response to H2O2, inhibition of hydrogen peroxide-induced intrinsic apoptotic signaling pathway, inhibition of intrinsic apoptotic signaling pathway in response to H2O2, inhibition of intrinsic apoptotic signaling pathway in response to hydrogen peroxide, down regulation of H2O2-induced intrinsic apoptotic signaling pathway, down-regulation of H2O2-induced intrinsic apoptotic signaling pathway, downregulation of H2O2-induced intrinsic apoptotic signaling pathway, inhibition of H2O2-induced intrinsic apoptotic signaling pathway, negative regulation of H2O2-induced intrinsic apoptotic signaling pathway